{
  "term_label": "regulation of postsynapse assembly",
  "gene_symbol": "ARHGAP33",
  "gene": "UniProtKB:O14559",
  "gene_name": "Rho GTPase-activating protein 33",
  "term_id": "GO:0150052"
}